pyrrolysine incorporation [GO:0030631] (biological process) References: PMID:11435424, PMID:17204561 Sources: RESID:AA0321 Definition: The incorporation of pyrrolysine, also known as lysine methylamine methyltransferase cofactor adduct, into a peptide; uses a special tRNA that recognizes the UAG codon as a modified lysine, rather than as a termination codon. Pyrrolysine may be synthesized as a free amino acid or synthesized from a lysine charged tRNA before its incorporation; it is not a posttranslational modification of peptidyl-lysine; this modification is found in several Methanosarcina methylamine methyltransferases. Also known as: lysine methylamine methyltransferase cofactor adduct incorporation, monomethylamine methyltransferase cofactor lysine adduct incorporation Relationships: is a type of GO:0006451